{
  "gene": "UniProtKB:Q9NVZ3",
  "gene_name": "Adaptin ear-binding coat-associated protein 2",
  "term_label": "vesicle-mediated transport",
  "term_id": "GO:0016192",
  "gene_symbol": "NECAP2"
}